{
  "term_label": "uniporter activity",
  "term_id": "GO:0015292",
  "gene_symbol": "MCU",
  "gene_name": "Calcium uniporter protein, mitochondrial",
  "gene": "UniProtKB:Q8NE86"
}